{
  "gene": "UniProtKB:Q92782",
  "gene_symbol": "DPF1",
  "gene_name": "Zinc finger protein neuro-d4",
  "term_label": "regulation of DNA-templated transcription",
  "term_id": "GO:0006355"
}